{
  "gene": "UniProtKB:P16435",
  "gene_name": "NADPH--cytochrome P450 reductase",
  "term_label": "NADPH-hemoprotein reductase activity",
  "term_id": "GO:0003958",
  "gene_symbol": "POR"
}